eukaryotic translation initiation factor 2 complex assembly [GO:1905143] (biological process) References: PMID:23775072 Sources: GOC:TermGenie, GO_REF:0000079 Relationships: is a type of protein-containing complex assembly [GO:0065003] Definition: The aggregation, arrangement and bonding together of a set of components to form an eukaryotic translation initiation factor 2 complex. Also known as: eIF-2 assembly, eIF-2 formation, eIF2 assembly, eIF2 formation, eukaryotic translation initiation factor 2 complex formation